{
  "gene": "UniProtKB:Q5TGI0",
  "term_id": "UNKNOWN:0002",
  "term_label": "Unknown biological process",
  "gene_name": "Failed axon connections homolog",
  "gene_symbol": "FAXC"
}